{
  "gene_name": "Zinc finger protein ZIC 5",
  "gene": "UniProtKB:Q96T25",
  "term_id": "GO:0006357",
  "term_label": "regulation of transcription by RNA polymerase II",
  "gene_symbol": "ZIC5"
}